negative regulation of forebrain neuron differentiation [GO:2000978] (biological process) Relationships: is_a negative regulation of neuron differentiation [GO:0045665]; is a type of GO:2000977; negatively regulates forebrain neuron differentiation [GO:0021879] Definition: Any process that stops, prevents or reduces the frequency, rate or extent of forebrain neuron differentiation. Sources: GOC:obol